{
  "term_id": "GO:0015671",
  "term_label": "oxygen transport",
  "gene_symbol": "HBD",
  "gene": "UniProtKB:P02042",
  "gene_name": "Hemoglobin subunit delta"
}